{
  "gene_name": "Macrophage mannose receptor 1",
  "term_id": "GO:0004888",
  "gene": "UniProtKB:P22897",
  "term_label": "transmembrane signaling receptor activity",
  "gene_symbol": "MRC1"
}